{
  "term_id": "GO:0048007",
  "gene_symbol": "CD1A",
  "term_label": "antigen processing and presentation, exogenous lipid antigen via MHC class Ib",
  "gene": "UniProtKB:P06126",
  "gene_name": "T-cell surface glycoprotein CD1a"
}